{
  "term_label": "glucosylceramide biosynthetic process",
  "gene_name": "Ceramide glucosyltransferase",
  "term_id": "GO:0006679",
  "gene": "UniProtKB:Q16739",
  "gene_symbol": "UGCG"
}